unencapsulated part of cell [GO:0097653] (CC) Relationships: is a type of cellular anatomical structure [GO:0110165]; has part intracellular anatomical structure [GO:0005622]; has part plasma membrane [GO:0005886] Sources: GOC:curators Definition: The part of a cell encompassing the intracellular environment and the plasma membrane; it excludes any external encapsulating structures. Also known as: non-encapsulated part of cell